{
  "gene": "UniProtKB:P59541",
  "term_id": "GO:0016020",
  "term_label": "membrane",
  "gene_name": "Taste receptor type 2 member 30",
  "gene_symbol": "TAS2R30"
}